{
  "term_id": "UNKNOWN:0001",
  "gene_symbol": "GPRASP3",
  "gene_name": "G protein-coupled receptor associated sorting protein 3",
  "term_label": "Unknown molecular function",
  "gene": "UniProtKB:Q6PI77"
}